{
  "gene_name": "Integrin alpha-7",
  "gene_symbol": "ITGA7",
  "term_label": "integrin complex",
  "gene": "UniProtKB:Q13683",
  "term_id": "GO:0008305"
}